{
  "gene_symbol": "RASL11B",
  "term_id": "UNKNOWN:0003",
  "gene": "UniProtKB:Q9BPW5",
  "gene_name": "Ras-like protein family member 11B",
  "term_label": "Unknown cellular component"
}